{
  "term_label": "proteolysis",
  "gene_name": "Serine protease HTRA1",
  "term_id": "GO:0006508",
  "gene_symbol": "HTRA1",
  "gene": "UniProtKB:Q92743"
}